mesonephric juxtaglomerulus cell development [GO:0061229] (biological process) Relationships: is a type of GO:0072142; BFO_0000050 mesonephric juxtaglomerulus cell differentiation [GO:0061207] Definition: The process whose specific outcome is the progression of a mesonephric juxtaglomerulus cell over time, from its formation to the mature structure. Sources: GOC:mtg_kidney_jan10